negative regulation of skeletal muscle tissue development [GO:0048642] (biological process) Definition: Any process that stops, prevents, or reduces the frequency, rate or extent of skeletal muscle tissue development. Also known as: down regulation of skeletal muscle development, down-regulation of skeletal muscle development, downregulation of skeletal muscle development, inhibition of skeletal muscle development Subtypes: negative regulation of branchiomeric skeletal muscle development [GO:0014713], negative regulation of extraocular skeletal muscle development [GO:0014726] Relationships: is a type of GO:0045843; is a type of GO:0048641; negatively regulates skeletal muscle tissue development [GO:0007519] Sources: GOC:go_curators